{
  "gene_symbol": "SMN2",
  "term_label": "nucleus",
  "gene": "UniProtKB:Q16637",
  "gene_name": "Survival motor neuron protein",
  "term_id": "GO:0005634"
}